{
  "gene_symbol": "SEMA3G",
  "term_id": "GO:0007411",
  "gene": "UniProtKB:Q9NS98",
  "gene_name": "Semaphorin-3G",
  "term_label": "axon guidance"
}